intracellular zinc ion homeostasis [GO:0006882] (biological process) Also known as: zinc homeostasis, cellular zinc ion homeostasis Relationships: is a type of intracellular monoatomic cation homeostasis [GO:0030003]; is a type of inorganic ion homeostasis [GO:0098771] Sources: GOC:ai, GOC:mah Definition: A homeostatic process involved in the maintenance of a steady state level of zinc ions within a cell.